negative regulation of axonemal microtubule depolymerization [GO:0007027] (biological process) Sources: GOC:dph, GOC:mah Definition: Any process that stops, prevents, or reduces the frequency, rate or extent of the depolymerization of the specialized microtubules of the axoneme. Relationships: is a type of negative regulation of microtubule depolymerization [GO:0007026]; is_a regulation of cytoplasmic microtubule depolymerization [GO:0010937]; is a type of negative regulation of cell projection organization [GO:0031345]; is a type of GO:0120035; negatively regulates axonemal microtubule depolymerization [GO:0060404] Also known as: axonemal microtubule stabilization, negative regulation of microtubule depolymerization in axoneme